imidazole-containing compound metabolic process [GO:0052803] (biological process) Also known as: imidazole metabolism Definition: The chemical reactions and pathways involving imidazoles, five-membered organic heterocycle containing two nitrogen atoms at positions 1 and 3, or any of its derivatives; compounds containing an imidazole skeleton. Subtypes: GO:0001692, L-histidine metabolic process [GO:0006547], iprodione metabolic process [GO:0018922], imidazole-containing compound catabolic process [GO:0052805] Relationships: is a type of metabolic process [GO:0008152] Sources: GOC:curators